methylisocitrate lyase activity [GO:0046421] (molecular function) Sources: EC:4.1.3.30, RHEA:16809 Definition: Catalysis of the reaction: (2S,3R)-3-hydroxybutane-1,2,3-tricarboxylate = pyruvate + succinate. Also known as: 2-methylisocitrate lyase activity, (2S,3R)-3-hydroxybutane-1,2,3-tricarboxylate pyruvate-lyase (succinate-forming), (2S,3R)-3-hydroxybutane-1,2,3-tricarboxylate pyruvate-lyase activity, MICL Relationships: is_a oxo-acid-lyase activity [GO:0016833]